{
  "term_label": "olfactory receptor activity",
  "gene_name": "Olfactory receptor 56A3",
  "gene_symbol": "OR56A3",
  "gene": "UniProtKB:Q8NH54",
  "term_id": "GO:0004984"
}